{
  "gene_name": "Patatin-like phospholipase domain-containing protein 4",
  "term_id": "GO:0004806",
  "gene_symbol": "PNPLA4",
  "term_label": "triacylglycerol lipase activity",
  "gene": "UniProtKB:P41247"
}